{
  "term_label": "cytoplasm",
  "gene_name": "F-box only protein 44",
  "gene_symbol": "FBXO44",
  "gene": "UniProtKB:Q9H4M3",
  "term_id": "GO:0005737"
}